{
  "gene_symbol": "PCDHGA10",
  "term_id": "GO:0007155",
  "gene_name": "Protocadherin gamma-A10",
  "gene": "UniProtKB:Q9Y5H3",
  "term_label": "cell adhesion"
}